{
  "gene_symbol": "TRBJ1-3",
  "gene_name": "T cell receptor beta joining 1-3",
  "term_label": "Unknown cellular component",
  "term_id": "UNKNOWN:0003",
  "gene": "UniProtKB:A0A0J9YWP8"
}